{
  "term_label": "plasma membrane",
  "gene": "UniProtKB:Q15382",
  "gene_symbol": "RHEB",
  "gene_name": "GTP-binding protein Rheb",
  "term_id": "GO:0005886"
}